non-proteinogenic amino acid biosynthetic process [GO:0170043] (biological process) Definition: The chemical reactions and pathways resulting in the formation of non-proteinogenic amino acids. Also known as: non-proteinogenic amino acid anabolism, non-proteinogenic amino acid formation, non-proteinogenic amino acid synthesis, non-proteinogenic biosynthesis Subtypes: GO:0006592, gamma-aminobutyric acid biosynthetic process [GO:0009449], citrulline biosynthetic process [GO:0019240], 4-hydroxyproline biosynthetic process [GO:0019472], beta-alanine biosynthetic process [GO:0019483], L-proline betaine biosynthetic process [GO:0019503], discadenine biosynthetic process [GO:0034268], 1-aminocyclopropane-1-carboxylate biosynthetic process [GO:0042218], GO:0046312, D-amino acid biosynthetic process [GO:0046437], hydroxylysine biosynthetic process [GO:0046947], L-beta-ethynylserine biosynthetic process [GO:0062142], L-propargylglycine biosynthetic process [GO:0062143], homocysteine biosynthetic process [GO:0071268], sarcosine biosynthetic process [GO:1901054], L-dopa biosynthetic process [GO:1903185], GO:1903560 Relationships: is a type of carboxylic acid biosynthetic process [GO:0046394]; is a type of non-proteinogenic amino acid metabolic process [GO:0170041] Sources: GOC:ew